{
  "term_id": "GO:0007189",
  "gene_name": "Melanocortin receptor 3",
  "gene_symbol": "MC3R",
  "gene": "UniProtKB:P41968",
  "term_label": "adenylate cyclase-activating G protein-coupled receptor signaling pathway"
}